{
  "gene_name": "Pancreatic lipase-related protein 3",
  "term_label": "cholesterol homeostasis",
  "gene": "UniProtKB:Q17RR3",
  "gene_symbol": "PNLIPRP3",
  "term_id": "GO:0042632"
}